{
  "term_label": "C-C chemokine binding",
  "gene_symbol": "CCR2",
  "gene_name": "C-C chemokine receptor type 2",
  "term_id": "GO:0019957",
  "gene": "UniProtKB:P41597"
}